positive regulation of thymine transport [GO:0035367] (biological process) Sources: GOC:bf, GOC:sl Definition: Any process that activates or increases the frequency, rate or extent of the directed movement of thymine, 5-methyluracil, into, out of or within a cell, or between cells, by means of some agent such as a transporter or pore. Relationships: is_a positive regulation of nucleobase-containing compound transport [GO:0032241]; is a type of regulation of thymine transport [GO:0035365]; positively regulates thymine transport [GO:0035364] Also known as: positive regulation of 5-methyluracil transport